regulation of maintenance of meiotic sister chromatid cohesion, centromeric [GO:2000709] (biological process) Also known as: regulation of maintenance of centromeric meiotic sister chromatin cohesion, regulation of maintenance of meiotic sister chromatin cohesion at centromere, regulation of maintenance of sister chromatin cohesion at centromere at meiosis I Relationships: is a type of regulation of maintenance of meiotic sister chromatid cohesion [GO:0034094]; is a type of regulation of centromeric sister chromatid cohesion [GO:0070602]; RO_0002211 GO:0035875 Definition: Any process that modulates the frequency, rate or extent of maintenance of meiotic sister chromatid cohesion in the centromeric region. Subtypes: negative regulation of maintenance of meiotic sister chromatid cohesion, centromeric [GO:2000710], positive regulation of maintenance of meiotic sister chromatid cohesion, centromeric [GO:2000711] Sources: GOC:mah